glycophagy [GO:0061723] (biological process) Relationships: is_a glycogen catabolic process [GO:0005980]; is_a macroautophagy [GO:0016236] Definition: The selective degradation of glycogen by macroautophagy. References: PMID:21893048 Sources: GOC:autophagy